paraflagellar rod [GO:0097740] (cellular component) Relationships: is_a supramolecular complex [GO:0099080]; is part of 9+2 motile cilium [GO:0097729] References: PMID:19879876, PMID:26199333, PMID:26688619 Sources: GOC:cilia Definition: A large lattice-like axial structure found in some flagellated protists which extends alongside the axoneme. Protein components of the paraflagellar rod are likely implicated, among other, in adenine nucleotide signaling and metabolism, and in calcium signaling. Also known as: PFR